{
  "term_label": "DNA binding",
  "gene_name": "DNA polymerase epsilon catalytic subunit A",
  "gene": "UniProtKB:Q07864",
  "term_id": "GO:0003677",
  "gene_symbol": "POLE"
}